{
  "term_id": "GO:0005886",
  "gene_name": "Protocadherin gamma-A4",
  "gene_symbol": "PCDHGA4",
  "gene": "UniProtKB:Q9Y5G9",
  "term_label": "plasma membrane"
}